{
  "term_label": "sensory perception of chemical stimulus",
  "gene_name": "Guanine nucleotide-binding protein G(olf) subunit alpha",
  "gene": "UniProtKB:P38405",
  "gene_symbol": "GNAL",
  "term_id": "GO:0007606"
}